{
  "gene": "UniProtKB:Q9HB07",
  "term_id": "GO:0005737",
  "term_label": "cytoplasm",
  "gene_name": "MYG1 exonuclease",
  "gene_symbol": "MYG1"
}